{
  "gene": "UniProtKB:O95072",
  "term_label": "meiotic sister chromatid cohesion",
  "term_id": "GO:0051177",
  "gene_name": "Meiotic recombination protein REC8 homolog",
  "gene_symbol": "REC8"
}